TRAIL production [GO:0032639] (biological process) Definition: The appearance of TRAIL due to biosynthesis or secretion following a cellular stimulus, resulting in an increase in its intracellular or extracellular levels. References: PMID:9311998 Sources: GOC:mah Relationships: is a type of tumor necrosis factor superfamily cytokine production [GO:0071706] Also known as: TRAIL biosynthetic process Regulation: regulated by regulation of TRAIL production [GO:0032679]; negatively regulated by negative regulation of TRAIL production [GO:0032719]; positively regulated by GO:0032759 Note: Note that this term is in the subset of terms that should not be used for direct gene product annotation. Instead, select one of the 'regulation' children terms.